negative regulation of attachment of spindle microtubules to kinetochore [GO:0051986] (biological process) Definition: Any process that stops, prevents, or reduces the frequency, rate or extent of the attachment of spindle microtubules to the kinetochore. Also known as: down regulation of attachment of spindle microtubules to kinetochore, down-regulation of attachment of spindle microtubules to kinetochore, downregulation of attachment of spindle microtubules to kinetochore, inhibition of attachment of spindle microtubules to kinetochore Sources: GOC:ai Subtypes: negative regulation of attachment of mitotic spindle microtubules to kinetochore [GO:1902424] Relationships: is_a negative regulation of chromosome segregation [GO:0051985]; is a type of GO:0051988; negatively regulates attachment of spindle microtubules to kinetochore [GO:0008608]